{
  "term_label": "centrosome localization",
  "gene_symbol": "NDE1",
  "term_id": "GO:0051642",
  "gene_name": "Nuclear distribution protein nudE homolog 1",
  "gene": "UniProtKB:Q9NXR1"
}